{
  "term_id": "UNKNOWN:0002",
  "term_label": "Unknown biological process",
  "gene_name": "BTB_POZ domain-containing protein KCTD9",
  "gene": "UniProtKB:Q7L273",
  "gene_symbol": "KCTD9"
}